{
  "term_id": "GO:0045944",
  "term_label": "positive regulation of transcription by RNA polymerase II",
  "gene_symbol": "NFE4",
  "gene_name": "Transcription factor NF-E4",
  "gene": "UniProtKB:Q86UQ8"
}